{
  "gene": "UniProtKB:P41222",
  "term_id": "UNKNOWN:0001",
  "gene_symbol": "PTGDS",
  "gene_name": "Prostaglandin-H2 D-isomerase",
  "term_label": "Unknown molecular function"
}